ascr#2 binding [GO:1904067] (molecular function) Definition: Binding to ascr#2. References: PMID:22665789 Sources: GOC:TermGenie, GOC:kmv, GO_REF:0000067 Relationships: is a type of carbohydrate derivative binding [GO:0097367]